glycylpeptide N-tetradecanoyltransferase activity [GO:0004379] (molecular function) Definition: Catalysis of the reaction: tetradecanoyl-CoA + glycyl-peptide = CoA + N-tetradecanoylglycyl-peptide. Relationships: is a type of N-acyltransferase activity [GO:0016410]; is a type of GO:0019107 Sources: EC:2.3.1.97 Also known as: N-myristoyltransferase activity, myristoyl-CoA-protein N-myristoyltransferase activity, myristoyl-coenzyme A:protein N-myristoyl transferase activity, myristoylating enzymes, peptide N-myristoyltransferase activity, peptide N-tetradecanoyltransferase activity, protein N-myristoyltransferase activity, tetradecanoyl-CoA:glycylpeptide N-tetradecanoyltransferase activity